{
  "gene": "UniProtKB:P0C1S8",
  "gene_symbol": "WEE2",
  "gene_name": "Wee1-like protein kinase 2",
  "term_label": "nucleus",
  "term_id": "GO:0005634"
}